UDP-glucose:4-aminobenzoate acylglucosyltransferase activity [GO:0080002] (molecular function) Relationships: is a type of GO:0035251 References: PMID:18385129 Also known as: UDP-glucose:p-aminobenzoate acylglucosyltransferase activity, UDP-glucose:p-aminobenzoate glucosyltransferase activity, UDP-glucose:pABA acylglucosyltransferase activity Definition: Catalysis of the reaction: 4-aminobenzoate + UDP-alpha-D-glucose = 1-O-(4-aminobenzoyl)-beta-D-glucose + UDP.